{
  "term_id": "GO:0005634",
  "term_label": "nucleus",
  "gene_name": "Zinc finger HIT domain-containing protein 3",
  "gene_symbol": "ZNHIT3",
  "gene": "UniProtKB:Q15649"
}